{
  "term_label": "Unknown cellular component",
  "gene_symbol": "C1orf216",
  "gene": "UniProtKB:Q8TAB5",
  "gene_name": "UPF0500 protein C1orf216",
  "term_id": "UNKNOWN:0003"
}